{
  "term_label": "Unknown cellular component",
  "term_id": "UNKNOWN:0003",
  "gene_name": "Pleckstrin homology domain-containing family A member 6",
  "gene": "UniProtKB:Q9Y2H5",
  "gene_symbol": "PLEKHA6"
}